{
  "gene": "UniProtKB:Q6ZR54",
  "gene_name": "Putative uncharacterized protein FLJ46641",
  "gene_symbol": "Q6ZR54",
  "term_id": "UNKNOWN:0001",
  "term_label": "Unknown molecular function"
}